regulation of somatostatin secretion [GO:0090273] (biological process) Definition: Any process that modulates the rate, frequency, extent of the regulated release of somatostatin from secretory granules in the D cells of the pancreas. Sources: GOC:BHF Relationships: is a type of regulation of peptide hormone secretion [GO:0090276]; regulates somatostatin secretion [GO:0070253] Subtypes: positive regulation of somatostatin secretion [GO:0090274], GO:0090275